{
  "term_id": "GO:0003713",
  "gene_symbol": "MED16",
  "gene": "UniProtKB:Q9Y2X0",
  "gene_name": "Mediator of RNA polymerase II transcription subunit 16",
  "term_label": "transcription coactivator activity"
}